{
  "gene_symbol": "FABP3",
  "gene": "UniProtKB:P05413",
  "term_label": "long-chain fatty acid transport",
  "term_id": "GO:0015909",
  "gene_name": "Fatty acid-binding protein, heart"
}